{
  "term_label": "calcium-dependent phospholipid binding",
  "gene_name": "Synaptotagmin-4",
  "gene_symbol": "SYT4",
  "gene": "UniProtKB:Q9H2B2",
  "term_id": "GO:0005544"
}